{
  "term_label": "skeletal system development",
  "term_id": "GO:0001501",
  "gene_name": "Hyaluronan and proteoglycan link protein 1",
  "gene": "UniProtKB:P10915",
  "gene_symbol": "HAPLN1"
}